complement component C5a binding [GO:0001856] (molecular function) Definition: Binding to a C5a product of the complement cascade. Sources: GOC:add, ISBN:0781735149 Relationships: is a type of complement binding [GO:0001848]